{
  "term_id": "GO:0004956",
  "gene_symbol": "PTGDR",
  "term_label": "prostaglandin D receptor activity",
  "gene": "UniProtKB:Q13258",
  "gene_name": "Prostaglandin D2 receptor"
}